{
  "term_label": "cytoplasm",
  "gene_name": "MAP_microtubule affinity-regulating kinase 4",
  "term_id": "GO:0005737",
  "gene": "UniProtKB:Q96L34",
  "gene_symbol": "MARK4"
}